{
  "gene": "UniProtKB:P08254",
  "gene_name": "Stromelysin-1",
  "gene_symbol": "MMP3",
  "term_label": "extracellular matrix organization",
  "term_id": "GO:0030198"
}